response to corticosterone [GO:0051412] (biological process) Definition: Any process that results in a change in state or activity of a cell or an organism (in terms of movement, secretion, enzyme production, gene expression, etc.) as a result of a corticosterone stimulus. Corticosterone is a 21 carbon steroid hormone of the corticosteroid type, produced in the cortex of the adrenal glands. In many species, corticosterone is the principal glucocorticoid, involved in regulation of fuel metabolism, immune reactions, and stress responses. References: PMID:15240347 Also known as: response to corticosterone stimulus Relationships: is a type of response to glucocorticoid [GO:0051384]; is a type of response to mineralocorticoid [GO:0051385]; is a type of response to alcohol [GO:0097305]; is a type of response to ketone [GO:1901654] Subtypes: cellular response to corticosterone stimulus [GO:0071386]